positive regulation of mononuclear cell proliferation [GO:0032946] (biological process) Definition: Any process that activates or increases the frequency, rate or extent of mononuclear cell proliferation. Sources: GOC:add Also known as: up regulation of mononuclear cell proliferation, up-regulation of mononuclear cell proliferation, upregulation of mononuclear cell proliferation, activation of mononuclear cell proliferation, positive regulation of PBMC proliferation, positive regulation of peripheral blood mononuclear cell proliferation, stimulation of mononuclear cell proliferation Relationships: is a type of regulation of mononuclear cell proliferation [GO:0032944]; is a type of positive regulation of leukocyte proliferation [GO:0070665]; positively regulates mononuclear cell proliferation [GO:0032943] Subtypes: positive regulation of lymphocyte proliferation [GO:0050671]